hamamelose kinase activity [GO:0047976] (molecular function) Sources: EC:2.7.1.102, RHEA:22796 Also known as: ATP/hamamelose 2'-phosphotransferase activity, ATP:D-hamamelose 2'-phosphotransferase activity, hamamelose kinase (phosphorylating), hamamelosekinase (ATP: hamamelose 2'-phosphotransferase) Definition: Catalysis of the reaction: D-hamamelose + ATP = D-hamamelose 2'-phosphate + ADP + 2 H+. Relationships: is a type of kinase activity [GO:0016301]; is a type of phosphotransferase activity, alcohol group as acceptor [GO:0016773]